{
  "term_id": "GO:0004674",
  "gene": "UniProtKB:Q13177",
  "gene_symbol": "PAK2",
  "gene_name": "Serine_threonine-protein kinase PAK 2",
  "term_label": "protein serine/threonine kinase activity"
}